{
  "gene_symbol": "TRIM15",
  "gene": "UniProtKB:Q9C019",
  "term_label": "ubiquitin protein ligase activity",
  "gene_name": "E3 ubiquitin-protein ligase TRIM15",
  "term_id": "GO:0061630"
}